{
  "gene_symbol": "CES5A",
  "gene": "UniProtKB:Q6NT32",
  "gene_name": "Carboxylesterase 5A",
  "term_id": "UNKNOWN:0002",
  "term_label": "Unknown biological process"
}